{
  "gene": "UniProtKB:P01854",
  "term_id": "GO:0003823",
  "term_label": "antigen binding",
  "gene_name": "Immunoglobulin heavy constant epsilon",
  "gene_symbol": "IGHE"
}